{
  "gene_name": "Nucleotide sugar transporter SLC35D1",
  "gene": "UniProtKB:Q9NTN3",
  "gene_symbol": "SLC35D1",
  "term_label": "antiporter activity",
  "term_id": "GO:0015297"
}